{
  "gene": "UniProtKB:Q15631",
  "gene_name": "Translin",
  "term_label": "RNA binding",
  "gene_symbol": "TSN",
  "term_id": "GO:0003723"
}